{
  "term_label": "DNA-binding transcription factor activity, RNA polymerase II-specific",
  "term_id": "GO:0000981",
  "gene_symbol": "EHF",
  "gene_name": "ETS homologous factor",
  "gene": "UniProtKB:Q9NZC4"
}